{
  "gene_symbol": "CPLX4",
  "gene_name": "Complexin-4",
  "term_label": "synaptic vesicle exocytosis",
  "gene": "UniProtKB:Q7Z7G2",
  "term_id": "GO:0016079"
}